zinc chaperone activity [GO:0140827] (molecular function) Relationships: is_a GO:0016530; has part zinc ion binding [GO:0008270] Definition: Binding to and delivering zinc ions to a target protein. References: PMID:35584675 Also known as: zinc carrier activity